negative regulation of metaphase/anaphase transition of meiotic cell cycle [GO:1902103] (biological process) Relationships: is_a negative regulation of meiotic cell cycle phase transition [GO:1901994]; is a type of negative regulation of metaphase/anaphase transition of cell cycle [GO:1902100]; is a type of regulation of metaphase/anaphase transition of meiotic cell cycle [GO:1902102]; is a type of negative regulation of meiotic chromosome separation [GO:1905133]; negatively regulates metaphase/anaphase transition of meiotic cell cycle [GO:0044785] Subtypes: meiotic spindle checkpoint signaling [GO:0044779], GO:1905187, negative regulation of metaphase/anaphase transition of meiosis II [GO:1905190] Definition: Any process that stops, prevents or reduces the frequency, rate or extent of metaphase/anaphase transition of meiotic cell cycle. Sources: GOC:TermGenie, GOC:mtg_cell_cycle Also known as: down regulation of meiotic metaphase/anaphase transition, down regulation of metaphase/anaphase transition of meiotic cell cycle, down-regulation of meiotic metaphase/anaphase transition, down-regulation of metaphase/anaphase transition of meiotic cell cycle, downregulation of meiotic metaphase/anaphase transition, downregulation of metaphase/anaphase transition of meiotic cell cycle, inhibition of meiotic metaphase/anaphase transition, negative regulation of meiotic metaphase/anaphase transition, inhibition of metaphase/anaphase transition of meiotic cell cycle